{
  "term_id": "GO:0005737",
  "term_label": "cytoplasm",
  "gene": "UniProtKB:P35638",
  "gene_name": "DNA damage-inducible transcript 3 protein",
  "gene_symbol": "DDIT3"
}